{
  "gene_name": "Deleted in esophageal cancer 1",
  "term_label": "Unknown molecular function",
  "gene": "UniProtKB:Q9P2X7",
  "gene_symbol": "DELEC1",
  "term_id": "UNKNOWN:0001"
}